{
  "gene_name": "Synaptotagmin-5",
  "term_label": "synaptic vesicle membrane",
  "gene": "UniProtKB:O00445",
  "term_id": "GO:0030672",
  "gene_symbol": "SYT5"
}